{
  "gene_symbol": "ZGRF1",
  "term_label": "double-strand break repair",
  "term_id": "GO:0006302",
  "gene": "UniProtKB:Q86YA3",
  "gene_name": "Protein ZGRF1"
}